{
  "term_label": "phosphatidylinositol 3-kinase binding",
  "gene": "UniProtKB:Q9Y4H2",
  "gene_symbol": "IRS2",
  "term_id": "GO:0043548",
  "gene_name": "Insulin receptor substrate 2"
}